{
  "gene": "UniProtKB:Q8NGA1",
  "gene_symbol": "OR1M1",
  "gene_name": "Olfactory receptor 1M1",
  "term_label": "plasma membrane",
  "term_id": "GO:0005886"
}